{
  "term_id": "GO:0140597",
  "gene": "UniProtKB:Q7L5D6",
  "term_label": "protein carrier chaperone",
  "gene_name": "Golgi to ER traffic protein 4 homolog",
  "gene_symbol": "GET4"
}